{
  "gene": "UniProtKB:Q9P2Y4",
  "term_id": "GO:0005634",
  "gene_symbol": "ZNF219",
  "gene_name": "Zinc finger protein 219",
  "term_label": "nucleus"
}